{
  "gene_name": "F-BAR and double SH3 domains protein 2",
  "term_id": "UNKNOWN:0001",
  "term_label": "Unknown molecular function",
  "gene_symbol": "FCHSD2",
  "gene": "UniProtKB:O94868"
}